complement activation, classical pathway [GO:0006958] (biological process) Definition: Any process involved in the activation of any of the steps of the classical pathway of the complement cascade which allows for the direct killing of microbes, the disposal of immune complexes, and the regulation of other immune processes. Sources: GOC:add, ISBN:0781735149 Also known as: complement cascade, classical pathway Relationships: is a type of complement activation [GO:0006956]; is part of GO:0002455 Regulation: regulated by regulation of complement activation, classical pathway [GO:0030450]; negatively regulated by negative regulation of complement activation, classical pathway [GO:0045959]; positively regulated by GO:0045960